{
  "term_id": "GO:0006003",
  "term_label": "fructose 2,6-bisphosphate metabolic process",
  "gene_symbol": "PFKFB1",
  "gene_name": "6-phosphofructo-2-kinase_fructose-2,6-bisphosphatase 1",
  "gene": "UniProtKB:P16118"
}